{
  "gene_name": "Killer cell immunoglobulin-like receptor 2DS1",
  "term_label": "immune receptor activity",
  "term_id": "GO:0140375",
  "gene": "UniProtKB:Q14954",
  "gene_symbol": "KIR2DS1"
}